symbiont-mediated suppression of host complement activation [GO:0042784] (biological process) Definition: A process by which a symbiont inhibits or disrupts the normal execution of the activation of complement in its host. The host is defined as the larger of the organisms involved in a symbiotic interaction. Relationships: is a type of GO:0052170 Also known as: active evasion of immune response of other organism via regulation of complement system of other organism involved in symbiotic interaction, suppression of complement activation by another organism, active immune evasion via modulation of host complement system, active immune evasion via regulation of host complement system, evasion of host immune response via modulation of host complement system, evasion of host immune response via regulation of host complement system, active evasion of host immune response via regulation of host complement system References: PMID:20194595, PMID:21191012, PMID:25830295, PMID:7745740 Subtypes: symbiont-mediated suppression of host complement activation by inactivation of complement proteins [GO:0141115], symbiont-mediated suppression of host complement activation by complement sequestering [GO:0141116], symbiont-mediated suppression of host complement activation by recruitment of complement control protein [GO:0141117], symbiont-mediated suppression of host complement activation by activation of host proteases [GO:0141203]